{
  "term_label": "Unknown cellular component",
  "gene_symbol": "SCRN3",
  "gene": "UniProtKB:Q0VDG4",
  "term_id": "UNKNOWN:0003",
  "gene_name": "Secernin-3"
}